{
  "gene_symbol": "WNT2",
  "term_label": "extracellular space",
  "term_id": "GO:0005615",
  "gene_name": "Protein Wnt-2",
  "gene": "UniProtKB:P09544"
}